{
  "term_label": "T cell differentiation involved in immune response",
  "term_id": "GO:0002292",
  "gene_name": "High affinity immunoglobulin epsilon receptor subunit gamma",
  "gene": "UniProtKB:P30273",
  "gene_symbol": "FCER1G"
}